{
  "gene_name": "Membrane-spanning 4-domains subfamily A member 6E",
  "term_id": "GO:0007166",
  "gene_symbol": "MS4A6E",
  "term_label": "cell surface receptor signaling pathway",
  "gene": "UniProtKB:Q96DS6"
}